{
  "term_label": "Unknown molecular function",
  "gene_name": "Selenoprotein H",
  "gene_symbol": "SELENOH",
  "term_id": "UNKNOWN:0001",
  "gene": "UniProtKB:Q8IZQ5"
}